{
  "term_id": "GO:0071598",
  "gene": "UniProtKB:Q7LC44",
  "gene_name": "Activity-regulated cytoskeleton-associated protein",
  "term_label": "neuronal ribonucleoprotein granule",
  "gene_symbol": "ARC"
}